{
  "term_id": "GO:0006646",
  "gene": "UniProtKB:Q9HBU6",
  "gene_symbol": "ETNK1",
  "gene_name": "Ethanolamine kinase 1",
  "term_label": "phosphatidylethanolamine biosynthetic process"
}